{
  "gene_symbol": "CACNG3",
  "term_label": "channel regulator activity",
  "term_id": "GO:0016247",
  "gene_name": "Voltage-dependent calcium channel gamma-3 subunit",
  "gene": "UniProtKB:O60359"
}